gastro-intestinal system smooth muscle contraction [GO:0014831] (BP) Subtypes: intestine smooth muscle contraction [GO:0014827], esophagus smooth muscle contraction [GO:0014846], stomach smooth muscle contraction [GO:0120063] Definition: A process in which force is generated within smooth muscle tissue, resulting in a change in muscle geometry. This process occurs in the gastro-intestinal system. Force generation involves a chemo-mechanical energy conversion step that is carried out by the actin/myosin complex activity, which generates force through ATP hydrolysis. The gastro-intestinal system generally refers to the digestive structures stretching from the mouth to anus, but does not include the accessory glandular organs (liver, pancreas and biliary tract). Regulation: regulated by GO:1904304; negatively regulated by negative regulation of gastro-intestinal system smooth muscle contraction [GO:1904305]; positively regulated by positive regulation of gastro-intestinal system smooth muscle contraction [GO:1904306] Relationships: is a type of GO:0006939 Sources: GOC:mtg_muscle, MA:0001523, MSH:D041981